axis elongation [GO:0003401] (biological process) Definition: The developmental growth that results in the elongation of a line that defines polarity or symmetry in an anatomical structure. Relationships: is a type of developmental growth involved in morphogenesis [GO:0060560] Subtypes: bud dilation involved in lung branching [GO:0060503], GO:0060602, GO:0090245 Also known as: elongation of an axis Sources: GOC:ascb_2009, GOC:dph, GOC:tb